{
  "term_id": "GO:0005794",
  "term_label": "Golgi apparatus",
  "gene": "UniProtKB:O60512",
  "gene_name": "Beta-1,4-galactosyltransferase 3",
  "gene_symbol": "B4GALT3"
}